{
  "term_label": "negative regulation of transforming growth factor beta receptor signaling pathway",
  "term_id": "GO:0030512",
  "gene_name": "Ski oncogene",
  "gene_symbol": "SKI",
  "gene": "UniProtKB:P12755"
}